{
  "gene_name": "Zinc finger protein with KRAB and SCAN domains 5",
  "gene_symbol": "ZKSCAN5",
  "term_id": "GO:0005634",
  "gene": "UniProtKB:Q9Y2L8",
  "term_label": "nucleus"
}